regulation of metanephric comma-shaped body morphogenesis [GO:2000006] (biological process) Definition: Any process that modulates the frequency, rate or extent of metanephric comma-shaped body morphogenesis. Sources: GOC:mtg_kidney_jan10, GOC:obol, GOC:yaf Relationships: is a type of regulation of animal organ morphogenesis [GO:2000027]; regulates GO:0072278 Subtypes: negative regulation of metanephric comma-shaped body morphogenesis [GO:2000007]